DNA-templated transcription open complex formation [GO:0001112] (BP) Subtypes: transcription open complex formation at RNA polymerase II promoter [GO:0001113] Also known as: promoter melting, DNA-dependent transcriptional open complex formation, DNA-templated transcriptional open complex formation, transcription open complex formation at bacterial-type RNA polymerase promoter, transcriptional open complex formation at bacterial-type RNA polymerase promoter Relationships: is a type of protein-DNA complex remodeling [GO:0001120]; is part of DNA-templated transcription initiation [GO:0006352] References: PMID:15020047, PMID:18280161 Sources: GOC:txnOH Definition: Any process involved in the melting of the DNA hybrid of the core promoter region within the transcriptional closed complex of an RNA polymerase preinitiation complex (PIC) to produce an open complex where the DNA duplex around the transcription initiation site is unwound to form the transcription bubble.